{
  "term_id": "GO:0005634",
  "term_label": "nucleus",
  "gene_name": "Zinc finger protein 783",
  "gene_symbol": "ZNF783",
  "gene": "UniProtKB:Q6ZMS7"
}